oxidoreductase activity, acting on the aldehyde or oxo group of donors, with a quinone or similar compound as acceptor [GO:0052738] (molecular function) Sources: EC:1.2.5.- Relationships: is a type of oxidoreductase activity, acting on the aldehyde or oxo group of donors [GO:0016903] Definition: Catalysis of an oxidation-reduction (redox) reaction in which an aldehyde or ketone (oxo) group acts as a hydrogen or electron donor and reduces a quinone or similar compound. Subtypes: pyruvate dehydrogenase (quinone) activity [GO:0052737]